carbohydrate transport [GO:0008643] (biological process) Definition: The directed movement of carbohydrate into, out of or within a cell, or between cells, by means of some agent such as a transporter or pore. Carbohydrates are a group of organic compounds based of the general formula Cx(H2O)y. Sources: GOC:ai Subtypes: oligosaccharide transport [GO:0015772], polysaccharide transport [GO:0015774], carbohydrate export [GO:0033231], carbohydrate transmembrane transport [GO:0034219] Also known as: sugar transport Relationships: is a type of transport [GO:0006810]